regulation of atrial cardiac muscle cell action potential [GO:0098910] (biological process) Subtypes: negative regulation of atrial cardiac muscle cell action potential [GO:1903948], positive regulation of atrial cardiac muscle cell action potential [GO:1903949] Definition: Any process that modulates the frequency, rate or extent of action potential creation, propagation or termination in an atrial cardiac muscle cell contributing to the regulation of its contraction. This typically occurs via modulation of the activity or expression of voltage-gated ion channels. Sources: GOC:BHF, GOC:mtg_cardiac_conduct_nov11 Relationships: is a type of regulation of cardiac muscle cell contraction [GO:0086004]; is_a regulation of cardiac muscle cell action potential [GO:0098901]; is a type of regulation of cardiac conduction [GO:1903779]; regulates atrial cardiac muscle cell action potential [GO:0086014]